{
  "term_label": "Unknown biological process",
  "gene": "UniProtKB:A0A0U1RRL7",
  "gene_name": "Protein MMP24OS",
  "gene_symbol": "MMP24OS",
  "term_id": "UNKNOWN:0002"
}